{
  "gene": "UniProtKB:A0A1B0GVM5",
  "gene_name": "Embryonic testis differentiation protein homolog C",
  "gene_symbol": "ETDC",
  "term_id": "UNKNOWN:0003",
  "term_label": "Unknown cellular component"
}